{
  "term_label": "methylmalonyl-CoA mutase activity",
  "term_id": "GO:0004494",
  "gene": "UniProtKB:P22033",
  "gene_name": "Methylmalonyl-CoA mutase, mitochondrial",
  "gene_symbol": "MMUT"
}